{
  "term_id": "GO:0043197",
  "gene_name": "Amyloid-beta A4 precursor protein-binding family A member 3",
  "term_label": "dendritic spine",
  "gene": "UniProtKB:O96018",
  "gene_symbol": "APBA3"
}